{
  "term_id": "GO:0006897",
  "gene_name": "Unconventional myosin-VIIb",
  "gene": "UniProtKB:Q6PIF6",
  "gene_symbol": "MYO7B",
  "term_label": "endocytosis"
}